{
  "gene_name": "Olfactory receptor 2F1",
  "term_id": "GO:0050911",
  "gene": "UniProtKB:Q13607",
  "gene_symbol": "OR2F1",
  "term_label": "detection of chemical stimulus involved in sensory perception of smell"
}